{
  "term_label": "cysteine dioxygenase activity",
  "gene": "UniProtKB:Q16878",
  "term_id": "GO:0017172",
  "gene_symbol": "CDO1",
  "gene_name": "Cysteine dioxygenase type 1"
}